negative regulation of glomerular mesangial cell proliferation [GO:0072125] (biological process) Definition: Any process that decreases the frequency, rate or extent of glomerular mesangial cell proliferation. Sources: GOC:mtg_kidney_jan10 Subtypes: GO:0072302, negative regulation of mesonephric glomerular mesangial cell proliferation [GO:2000091] Relationships: is a type of regulation of glomerular mesangial cell proliferation [GO:0072124]; is a type of negative regulation of cell proliferation involved in kidney development [GO:1901723]; negatively regulates glomerular mesangial cell proliferation [GO:0072110]